regulation of translation in response to endoplasmic reticulum stress [GO:0036490] (biological process) Also known as: regulation of translation in response to ER stress References: PMID:14676213, PMID:16835242 Sources: GOC:PARL, GOC:bf Relationships: is a type of GO:0043555; is part of GO:0034976 Definition: Modulation of the frequency, rate or extent of translation as a result of endoplasmic reticulum stress. Subtypes: regulation of translation initiation in response to endoplasmic reticulum stress [GO:0036491], positive regulation of translation in response to endoplasmic reticulum stress [GO:0036493], negative regulation of translation in response to endoplasmic reticulum stress [GO:1902010]